3-(3-hydroxyphenyl)propanoate catabolic process [GO:1901794] (BP) Definition: The chemical reactions and pathways resulting in the breakdown of 3-(3-hydroxyphenyl)propanoate. References: PMID:10537203 Sources: GOC:TermGenie, GOC:yaf, MetaCyc:PWY0-1277, UniPathway:UPA00835 Also known as: 3-(3-hydroxyphenyl)propanoate breakdown, 3-(3-hydroxyphenyl)propanoate catabolism, 3-(3-hydroxyphenyl)propanoate degradation Relationships: is a type of monocarboxylic acid catabolic process [GO:0072329]